medial layer of collagen and cuticulin-based cuticle extracellular matrix [GO:0060109] (cellular component) Sources: GOC:dph, GOC:kmv, ISSN:15518507 Also known as: medial layer struts Definition: The fluid-filled cuticle layer that lies between the cortical and basal layers and is characterized by the presence of regularly spaced columnar struts that lie on either side of the annular furrows and link the two surrounding layers. In C. elegans, a defined medial layer is found only in adult animals. Relationships: is a type of GO:0110165; is part of cuticular extracellular matrix [GO:0060102]